{
  "gene_symbol": "RPL24",
  "term_label": "cytoplasmic translation",
  "gene_name": "Large ribosomal subunit protein eL24",
  "term_id": "GO:0002181",
  "gene": "UniProtKB:P83731"
}